{
  "term_label": "Unknown biological process",
  "gene": "UniProtKB:Q8NGI7",
  "gene_name": "Olfactory receptor 10V1",
  "term_id": "UNKNOWN:0002",
  "gene_symbol": "OR10V1"
}